apoptotic process in bone marrow cell [GO:0071839] (biological process) Also known as: bone marrow cell apoptosis, bone marrow cell programmed cell death by apoptosis, killing of bone marrow cells, programmed cell death of bone marrow cells by apoptosis, programmed cell death, bone marrow cells, apoptosis in bone marrow References: PMID:17063141 Sources: GOC:mah, GOC:mtg_apoptosis Regulation: regulated by regulation of apoptotic process in bone marrow cell [GO:0071865]; negatively regulated by negative regulation of apoptotic process in bone marrow cell [GO:0071866]; positively regulated by positive regulation of apoptotic process in bone marrow cell [GO:0120132] Relationships: is a type of apoptotic process [GO:0006915] Definition: The apoptotic process in cells in the bone marrow.